{
  "gene_symbol": "EDNRB",
  "gene_name": "Endothelin receptor type B",
  "term_label": "endothelin receptor signaling pathway",
  "term_id": "GO:0086100",
  "gene": "UniProtKB:P24530"
}